tagatose-6-phosphate kinase activity [GO:0009024] (molecular function) Sources: EC:2.7.1.144 Definition: Catalysis of the reaction: ATP + D-tagatose 6-phosphate = ADP + D-tagatose 1,6-bisphosphate. Relationships: is a type of kinase activity [GO:0016301]; is a type of GO:0016773 Also known as: ATP:D-tagatose-6-phosphate 1-phosphotransferase activity, phosphotagatokinase activity